{
  "gene_name": "Neurotrophin-4",
  "gene_symbol": "NTF4",
  "term_id": "GO:0021675",
  "gene": "UniProtKB:P34130",
  "term_label": "nerve development"
}